{
  "term_label": "ERAD pathway",
  "gene": "UniProtKB:Q9NR34",
  "gene_name": "Mannosyl-oligosaccharide 1,2-alpha-mannosidase IC",
  "term_id": "GO:0036503",
  "gene_symbol": "MAN1C1"
}